{
  "gene": "UniProtKB:H7C350",
  "gene_symbol": "CCDC188",
  "gene_name": "Coiled-coil domain-containing protein 188",
  "term_label": "Unknown biological process",
  "term_id": "UNKNOWN:0002"
}